regulation of vascular associated smooth muscle contraction [GO:0003056] (biological process) Also known as: regulation of vascular smooth muscle contraction Subtypes: regulation of vein smooth muscle contraction [GO:0062086], GO:1904694, positive regulation of vascular associated smooth muscle contraction [GO:1904695], regulation of artery smooth muscle contraction [GO:1905654] Sources: GOC:mtg_cardio, GOC:mtg_sensu, GOC:rl Definition: Any process that increases the frequency, rate or extent of vascular smooth muscle contraction. Relationships: is a type of regulation of smooth muscle contraction [GO:0006940]; is a type of regulation of vasoconstriction [GO:0019229]; regulates vascular associated smooth muscle contraction [GO:0014829]